{
  "gene_name": "Tumor necrosis factor receptor superfamily member 14",
  "gene_symbol": "TNFRSF14",
  "term_label": "defense response to Gram-positive bacterium",
  "term_id": "GO:0050830",
  "gene": "UniProtKB:Q92956"
}